{
  "term_label": "Unknown biological process",
  "gene": "UniProtKB:A0A0G2JPN4",
  "gene_symbol": "A0A0G2JPN4",
  "term_id": "UNKNOWN:0002",
  "gene_name": "Uncharacterized protein"
}